{
  "term_label": "glycerophospholipid catabolic process",
  "term_id": "GO:0046475",
  "gene": "UniProtKB:Q3MJ16",
  "gene_symbol": "PLA2G4E",
  "gene_name": "Cytosolic phospholipase A2 epsilon"
}